{
  "term_id": "GO:0005737",
  "gene_name": "Membrane-associated phosphatidylinositol transfer protein 2",
  "gene_symbol": "PITPNM2",
  "gene": "UniProtKB:Q9BZ72",
  "term_label": "cytoplasm"
}